{
  "term_id": "GO:0003723",
  "term_label": "RNA binding",
  "gene": "UniProtKB:Q6NWY9",
  "gene_symbol": "PRPF40B",
  "gene_name": "Pre-mRNA-processing factor 40 homolog B"
}